{
  "term_id": "GO:0031012",
  "gene": "UniProtKB:Q99218",
  "gene_name": "Amelogenin, Y isoform",
  "term_label": "extracellular matrix",
  "gene_symbol": "AMELY"
}